positive regulation of early stripe melanocyte differentiation [GO:0050948] (biological process) Relationships: is a type of positive regulation of melanocyte differentiation [GO:0045636]; is a type of regulation of early stripe melanocyte differentiation [GO:0050939]; positively regulates early stripe melanocyte differentiation [GO:0050933] Definition: Any process that activates or increases the frequency, rate or extent of early stripe melanocyte differentiation. Also known as: positive regulation of early stripe melanophore differentiation, up regulation of early stripe melanocyte differentiation, up-regulation of early stripe melanocyte differentiation, upregulation of early stripe melanocyte differentiation, activation of early stripe melanocyte differentiation, stimulation of early stripe melanocyte differentiation Sources: GOC:ai